{
  "term_label": "cytoplasm",
  "gene_symbol": "TXNRD1",
  "gene_name": "Thioredoxin reductase 1, cytoplasmic",
  "gene": "UniProtKB:Q16881",
  "term_id": "GO:0005737"
}